negative regulation of amine catabolic process [GO:0033242] (biological process) Sources: GOC:mah Relationships: is a type of negative regulation of catabolic process [GO:0009895]; is_a GO:0033239; is a type of GO:0033241; negatively regulates amine catabolic process [GO:0009310] Subtypes: GO:1900082 Also known as: negative regulation of amine breakdown, negative regulation of amine catabolism, negative regulation of amine degradation, negative regulation of cellular amine catabolic process Definition: Any process that stops, prevents, or reduces the frequency, rate or extent of the chemical reactions and pathways leading to the breakdown of amines.